{
  "term_id": "GO:0004984",
  "gene_name": "Olfactory receptor 13C8",
  "term_label": "olfactory receptor activity",
  "gene": "UniProtKB:Q8NGS7",
  "gene_symbol": "OR13C8"
}